protein palmitoleylation [GO:0045234] (biological process) Also known as: protein amino acid palmitoleylation Definition: The covalent attachment of a palmitoleyl group to a protein. Sources: GOC:ai Relationships: is_a protein lipidation [GO:0006497]; is a type of protein acylation [GO:0043543]